{
  "term_label": "DNA-binding transcription factor activity, RNA polymerase II-specific",
  "gene_name": "Transcription factor NF-E2 45 kDa subunit",
  "gene": "UniProtKB:Q16621",
  "term_id": "GO:0000981",
  "gene_symbol": "NFE2"
}